{
  "gene": "UniProtKB:A0JD32",
  "term_id": "UNKNOWN:0001",
  "term_label": "Unknown molecular function",
  "gene_symbol": "TRAV38-2DV8",
  "gene_name": "T cell receptor alpha variable 38-2_delta variable 8"
}